{
  "term_label": "endoplasmic reticulum",
  "gene": "UniProtKB:Q6UXD5",
  "gene_symbol": "SEZ6L2",
  "term_id": "GO:0005783",
  "gene_name": "Seizure 6-like protein 2"
}